{
  "gene_symbol": "DPCD",
  "term_label": "Unknown molecular function",
  "gene_name": "Protein DPCD",
  "gene": "UniProtKB:Q9BVM2",
  "term_id": "UNKNOWN:0001"
}